ocellus photoreceptor cell differentiation [GO:0042705] (biological process) Definition: The process in which a relatively unspecialized cell acquires specialized features of a photoreceptor cell found in the ocellus. Relationships: is a type of photoreceptor cell differentiation [GO:0046530] Sources: GOC:go_curators